{
  "gene_symbol": "GBP2",
  "gene": "UniProtKB:P32456",
  "gene_name": "Guanylate-binding protein 2",
  "term_label": "cytoplasmic vesicle",
  "term_id": "GO:0031410"
}